{
  "gene_symbol": "GP2",
  "gene_name": "Pancreatic secretory granule membrane major glycoprotein GP2",
  "term_label": "apical plasma membrane",
  "gene": "UniProtKB:P55259",
  "term_id": "GO:0016324"
}